{
  "term_label": "Unknown cellular component",
  "term_id": "UNKNOWN:0003",
  "gene_name": "Keratin-like protein KRT222",
  "gene": "UniProtKB:Q8N1A0",
  "gene_symbol": "KRT222"
}